{
  "term_label": "mitochondrion",
  "gene_symbol": "PDSS1",
  "gene": "UniProtKB:Q5T2R2",
  "term_id": "GO:0005739",
  "gene_name": "All trans-polyprenyl-diphosphate synthase PDSS1"
}